{
  "term_id": "UNKNOWN:0002",
  "gene_symbol": "TMEM9",
  "gene_name": "Proton-transporting V-type ATPase complex assembly regulator TMEM9",
  "term_label": "Unknown biological process",
  "gene": "UniProtKB:Q9P0T7"
}